re-entry into mitotic cell cycle [GO:0000320] (biological process) Sources: GOC:krc Subtypes: re-entry into mitotic cell cycle after pheromone arrest [GO:0000321] Relationships: is a type of GO:0022402 Definition: The resumption of the mitotic cell division cycle by cells that were in a quiescent or other non-dividing state.